GDP-Man:Man(1)GlcNAc(2)-PP-Dol alpha-1,3-mannosyltransferase activity [GO:0004378] (molecular function) Relationships: is a type of GO:0000033; is a type of GO:0120562 Sources: RHEA:29515 Also known as: GDP-D-mannose:D-Man-beta-(1->4)-D-GlcNAc-beta-(1->4)-D-GlcNAc-diphosphodolichol 3-alpha-mannosyltransferase activity, GDP-mannose-oligosaccharide-lipid mannosyltransferase II, GDP-mannose:glycolipid 1,3-alpha-D-mannosyltransferase activity, glycolipid 3-alpha-mannosyltransferase activity, guanosine diphosphomannose-oligosaccharide-lipid II mannosyltransferase activity, mannosyltransferase II activity Definition: Catalysis of the reaction: a beta-D-Man-(1->4)-beta-D-GlcNAc-(1->4)-alpha-D-GlcNAc-diphospho-di-trans,poly-cis-dolichol + GDP-alpha-D-mannose = an alpha-D-Man-(1->3)-beta-D-Man-(1->4)-beta-D-GlcNAc-(1->4)-alpha-D-GlcNAc-diphospho-di-trans,poly-cis-dolichol + GDP + H+.